{
  "gene": "UniProtKB:O76064",
  "gene_name": "E3 ubiquitin-protein ligase RNF8",
  "term_id": "GO:0061630",
  "gene_symbol": "RNF8",
  "term_label": "ubiquitin protein ligase activity"
}